post-embryonic plant organ morphogenesis [GO:0090697] (biological process) Subtypes: post-embryonic root morphogenesis [GO:0010101], GO:0048444 Definition: Morphogenesis, during the post-embryonic phase, of a plant tissue or tissues that work together to perform a specific function or functions. Morphogenesis pertains to process in which anatomical structures are generated and organized. Organs are commonly observed as visibly distinct structures, but may also exist as loosely associated clusters of cells that work together to perform a specific function or functions. Relationships: is a type of post-embryonic plant morphogenesis [GO:0090698]; is a type of plant organ morphogenesis [GO:1905392]; is part of post-embryonic plant organ development [GO:0090696] Sources: GOC:tb